{
  "gene": "UniProtKB:Q9NXR1",
  "term_id": "GO:0007059",
  "gene_symbol": "NDE1",
  "gene_name": "Nuclear distribution protein nudE homolog 1",
  "term_label": "chromosome segregation"
}